{
  "term_id": "GO:0016020",
  "gene_name": "Prostaglandin F2 receptor negative regulator",
  "term_label": "membrane",
  "gene": "UniProtKB:Q9P2B2",
  "gene_symbol": "PTGFRN"
}